retinal cone cell differentiation [GO:0042670] (biological process) Sources: GOC:go_curators Definition: The process in which a relatively unspecialized cell acquires the specialized features of a retinal cone cell. Relationships: is a type of GO:0060219